{
  "gene": "UniProtKB:Q9H521",
  "term_id": "UNKNOWN:0001",
  "gene_symbol": "Q9H521",
  "term_label": "Unknown molecular function",
  "gene_name": "Putative uncharacterized protein LOC645739"
}